primary prostatic bud elongation [GO:0060516] (biological process) Also known as: prostate bud elongation, prostate bud elongation involved in prostate morphogenesis Relationships: is a type of branch elongation of an epithelium [GO:0060602]; is a type of prostate gland morphogenetic growth [GO:0060737]; is a type of prostate gland epithelium morphogenesis [GO:0060740] References: PMID:18977204 Sources: GOC:dph Definition: The increase in size of the prostatic bud as it forms.